ether biosynthetic process [GO:1901503] (BP) Subtypes: DIF-1 biosynthetic process [GO:0031148], ferulate biosynthetic process [GO:0033495], GO:0033497, vanillin biosynthetic process [GO:0042189], eugenol biosynthetic process [GO:0042855], novobiocin biosynthetic process [GO:0043642], glycerol ether biosynthetic process [GO:0046504], vomitoxin biosynthetic process [GO:0106110], GO:0140654, (M)-viriditoxin biosynthetic process [GO:0140783], GO:0140872, diorcinol biosynthetic process [GO:1900572], GO:1900578, violaceol I biosynthetic process [GO:1900590], violaceol II biosynthetic process [GO:1900593], GO:1900766, fonsecin biosynthetic process [GO:1900769], GO:1900799, scopolamine biosynthetic process [GO:1900991], spheroidene biosynthetic process [GO:1901180], (-)-microperfuranone biosynthetic process [GO:1901512], (-)-pinoresinol biosynthetic process [GO:1901599], leukotriene A4 biosynthetic process [GO:1901753], pentalenolactone biosynthetic process [GO:1901780], GO:1901803, GO:1901833, fumagillin biosynthetic process [GO:1902086], GO:1902126, GO:1902132, GO:1902181 Relationships: is a type of GO:0009058 Sources: GOC:TermGenie, GOC:pr Also known as: ether anabolism, ether biosynthesis, ether formation, ether synthesis Definition: The chemical reactions and pathways resulting in the formation of ether.